{
  "gene_name": "Homeobox protein goosecoid-2",
  "gene": "UniProtKB:O15499",
  "term_label": "DNA-binding transcription factor activity, RNA polymerase II-specific",
  "term_id": "GO:0000981",
  "gene_symbol": "GSC2"
}